{
  "gene_symbol": "YTHDC1",
  "gene": "UniProtKB:Q96MU7",
  "gene_name": "YTH domain-containing protein 1",
  "term_id": "GO:0005654",
  "term_label": "nucleoplasm"
}